{
  "gene": "UniProtKB:Q8NHS3",
  "term_id": "GO:0005765",
  "gene_symbol": "MFSD8",
  "gene_name": "Major facilitator superfamily domain-containing protein 8",
  "term_label": "lysosomal membrane"
}